{
  "gene_symbol": "HOXB13",
  "gene_name": "Homeobox protein Hox-B13",
  "term_id": "GO:0000978",
  "gene": "UniProtKB:Q92826",
  "term_label": "RNA polymerase II cis-regulatory region sequence-specific DNA binding"
}